negative regulation of somitomeric trunk muscle development [GO:0014710] (biological process) Definition: Any process that stops, prevents, or reduces the frequency, rate or extent of somitomeric trunk muscle development. The somitomeric trunk muscle is derived from somitomeric mesoderm. The muscle begins its development with the differentiation of the muscle cells and ends with the mature muscle. Relationships: is a type of GO:0014708; is a type of GO:0048635; negatively regulates GO:0002075 Sources: GOC:mtg_muscle